{
  "term_label": "negative regulation of transcription elongation by RNA polymerase II",
  "gene_name": "Negative elongation factor C_D",
  "term_id": "GO:0034244",
  "gene_symbol": "NELFCD",
  "gene": "UniProtKB:Q8IXH7"
}